{
  "term_label": "lipoprotein metabolic process",
  "gene_name": "Oxidized low-density lipoprotein receptor 1",
  "gene_symbol": "OLR1",
  "term_id": "GO:0042157",
  "gene": "UniProtKB:P78380"
}